regulation of endocytosis [GO:0030100] (biological process) Definition: Any process that modulates the frequency, rate or extent of endocytosis. Sources: GOC:go_curators Relationships: is a type of regulation of cellular component organization [GO:0051128]; is a type of regulation of vesicle-mediated transport [GO:0060627]; regulates GO:0006897 Subtypes: GO:0045806, positive regulation of endocytosis [GO:0045807], regulation of receptor-mediated endocytosis [GO:0048259], GO:0048548, regulation of phagocytosis [GO:0050764], GO:0051600, regulation of synaptic vesicle endocytosis [GO:1900242], regulation of ubiquitin-dependent endocytosis [GO:2000395], regulation of caveolin-mediated endocytosis [GO:2001286]